{
  "term_id": "GO:0006955",
  "gene_name": "Probable non-functional immunoglobulin kappa variable 2D-24",
  "gene": "UniProtKB:A0A075B6R9",
  "gene_symbol": "IGKV2D-24",
  "term_label": "immune response"
}